mineralocorticoid secretion [GO:0035931] (BP) Sources: GOC:sl Subtypes: aldosterone secretion [GO:0035932] Regulation: regulated by regulation of mineralocorticoid secretion [GO:2000855]; negatively regulated by negative regulation of mineralocorticoid secretion [GO:2000856]; positively regulated by positive regulation of mineralocorticoid secretion [GO:2000857] Definition: The regulated release of any mineralocorticoid into the circulatory system. Mineralocorticoids are a class of steroid hormones that regulate water and electrolyte metabolism. Relationships: is a type of corticosteroid hormone secretion [GO:0035930]